{
  "gene_name": "Dihydrofolate reductase",
  "term_id": "GO:0004146",
  "gene": "UniProtKB:P00374",
  "gene_symbol": "DHFR",
  "term_label": "dihydrofolate reductase activity"
}